plasma membrane repair [GO:0001778] (BP) References: PMID:12925704 Sources: GOC:add Relationships: is_a GO:0007009; is part of wound healing [GO:0042060] Regulation: regulated by regulation of plasma membrane repair [GO:1905684]; negatively regulated by negative regulation of plasma membrane repair [GO:1905685]; positively regulated by positive regulation of plasma membrane repair [GO:1905686] Definition: The resealing of a cell plasma membrane after cellular wounding due to, for instance, mechanical stress.